{
  "gene": "UniProtKB:O15131",
  "gene_name": "Importin subunit alpha-6",
  "gene_symbol": "KPNA5",
  "term_label": "NLS-dependent protein nuclear import complex",
  "term_id": "GO:0042564"
}